type III intermediate filament [GO:0045098] (cellular component) Definition: A type of intermediate filament, typically made up of one or more of the proteins vimentin, desmin, glial fibrillary acidic protein (GFAP), and peripherin. Unlike the keratins, the type III proteins can form both homo- and heteropolymeric IF filaments. Sources: ISBN:0716731363 Also known as: desmin, glial fibrillary acidic protein, peripherin, type III intermediate filament associated protein, vimentin Relationships: is a type of intermediate filament [GO:0005882]